{
  "gene_symbol": "HR",
  "gene_name": "Lysine-specific demethylase hairless",
  "term_label": "histone deacetylase complex",
  "term_id": "GO:0000118",
  "gene": "UniProtKB:O43593"
}